positive regulation of interleukin-17A production [GO:0150153] (biological process) Relationships: is_a positive regulation of interleukin-17 production [GO:0032740]; is a type of GO:0150151; positively regulates interleukin-17A production [GO:0097087] Sources: GOC:aruk Also known as: positive regulation of interleukin-17A biosynthetic process Definition: Any process that activates or increases the frequency, rate or extent of interleukin-17A production.